{
  "gene_symbol": "TTC36",
  "term_label": "tyrosine metabolic process",
  "gene": "UniProtKB:A6NLP5",
  "gene_name": "Tetratricopeptide repeat protein 36",
  "term_id": "GO:0006570"
}